{
  "gene": "UniProtKB:Q9BT67",
  "term_label": "positive regulation of protein ubiquitination",
  "gene_name": "NEDD4 family-interacting protein 1",
  "term_id": "GO:0031398",
  "gene_symbol": "NDFIP1"
}